{
  "term_id": "UNKNOWN:0001",
  "gene_name": "Adaptin ear-binding coat-associated protein 1",
  "gene": "UniProtKB:Q8NC96",
  "term_label": "Unknown molecular function",
  "gene_symbol": "NECAP1"
}